(3R)-hydroxyacyl-[acyl-carrier-protein] dehydratase activity [GO:0019171] (molecular function) Also known as: 3-hydroxyacyl-[acyl-carrier-protein] dehydratase activity, 3-hydroxyacyl-ACP dehydratase activity, 3-hydroxyacyl-[acyl-carrier protein] dehydratase activity, (3R)-3-hydroxyacyl-[acyl-carrier-protein] dehydratase activity Relationships: is a type of hydro-lyase activity [GO:0016836] Sources: RHEA:13097 Definition: Catalysis of the reaction: a (3R)-hydroxyacyl-[acyl-carrier-protein] = a (2E)-enoyl-[acyl-carrier-protein] + H2O.